{
  "gene": "UniProtKB:Q9BYZ6",
  "gene_name": "Rho-related BTB domain-containing protein 2",
  "term_label": "cytoplasmic vesicle",
  "gene_symbol": "RHOBTB2",
  "term_id": "GO:0031410"
}